cellular response to salicylic acid stimulus [GO:0071446] (biological process) Sources: GOC:mah Relationships: is a type of response to salicylic acid [GO:0009751]; is a type of cellular response to oxygen-containing compound [GO:1901701] Definition: Any process that results in a change in state or activity of a cell (in terms of movement, secretion, enzyme production, gene expression, etc.) as a result of a salicylic acid stimulus. Also known as: cellular response to salicylate stimulus